{
  "gene_symbol": "CNIH1",
  "term_id": "UNKNOWN:0003",
  "gene_name": "Protein cornichon homolog 1",
  "gene": "UniProtKB:O95406",
  "term_label": "Unknown cellular component"
}